{
  "gene_symbol": "SLC30A9",
  "term_label": "Unknown molecular function",
  "gene_name": "Proton-coupled zinc antiporter SLC30A9, mitochondrial",
  "gene": "UniProtKB:Q6PML9",
  "term_id": "UNKNOWN:0001"
}